{
  "gene": "UniProtKB:P53350",
  "gene_symbol": "PLK1",
  "gene_name": "Serine_threonine-protein kinase PLK1",
  "term_label": "spindle pole",
  "term_id": "GO:0000922"
}